{
  "term_id": "UNKNOWN:0002",
  "gene": "UniProtKB:P49901",
  "gene_name": "Sperm mitochondrial-associated cysteine-rich protein",
  "gene_symbol": "SMCP",
  "term_label": "Unknown biological process"
}